{
  "gene_name": "Large ribosomal subunit protein uL13",
  "gene_symbol": "RPL13A",
  "gene": "UniProtKB:P40429",
  "term_label": "negative regulation of translation",
  "term_id": "GO:0017148"
}